{
  "term_id": "GO:0015629",
  "gene_symbol": "PARVA",
  "gene_name": "Alpha-parvin",
  "gene": "UniProtKB:Q9NVD7",
  "term_label": "actin cytoskeleton"
}